{
  "gene_name": "DNA dC-dU-editing enzyme APOBEC-3A",
  "term_id": "GO:0070383",
  "term_label": "DNA cytosine deamination",
  "gene_symbol": "APOBEC3A",
  "gene": "UniProtKB:P31941"
}